negative regulation of zinc ion transmembrane import [GO:0071584] (biological process) Sources: GOC:BHF, GOC:mah Relationships: is_a GO:0071581; is a type of negative regulation of zinc ion transmembrane transport [GO:0071583]; negatively regulates zinc ion import across plasma membrane [GO:0071578] Definition: Any process that stops, prevents, or reduces the frequency, rate or extent of zinc ion import.